{
  "gene_symbol": "CYP4V2",
  "gene_name": "Cytochrome P450 4V2",
  "term_id": "UNKNOWN:0002",
  "term_label": "Unknown biological process",
  "gene": "UniProtKB:Q6ZWL3"
}